ferrochelatase activity [GO:0004325] (molecular function) Relationships: is a type of lyase activity [GO:0016829] Definition: Catalysis of the reaction: heme B (protoheme) + H+ = Fe(2+) + protoporphyrin IX. Subtypes: GO:0051266 Also known as: heme synthase activity, heme synthetase activity, iron chelatase activity, ferro-protoporphyrin chelatase activity, protoheme ferro-lyase (protoporphyrin-forming), protoheme ferro-lyase activity, protoheme ferrolyase activity Sources: RHEA:22584